{
  "gene_name": "ARF GTPase-activating protein GIT1",
  "gene": "UniProtKB:Q9Y2X7",
  "term_id": "GO:0007420",
  "term_label": "brain development",
  "gene_symbol": "GIT1"
}